{
  "gene_name": "UDP-N-acetylhexosamine pyrophosphorylase",
  "gene_symbol": "UAP1",
  "term_label": "UDP-N-acetylglucosamine biosynthetic process",
  "term_id": "GO:0006048",
  "gene": "UniProtKB:Q16222"
}